intermediate conductance calcium-activated potassium channel activity [GO:0022894] (molecular function) Relationships: is a type of calcium-activated potassium channel activity [GO:0015269] Definition: Enables the transmembrane transfer of potassium by a channel with a unit conductance of 20 to 85 picoSiemens that opens in response to stimulus by internal calcium ions. Intermediate conductance calcium-activated potassium channels are more sensitive to calcium than are large conductance calcium-activated potassium channels. Transport by a channel involves catalysis of facilitated diffusion of a solute (by an energy-independent process) involving passage through a transmembrane aqueous pore or channel, without evidence for a carrier-mediated mechanism. Sources: GOC:mtg_transport, OMIM:602754 Also known as: IK KCa channels, IK calcium-activated potassium channel activity, intermediate conductance KCa channels